{
  "term_label": "regulation of postsynaptic membrane neurotransmitter receptor levels",
  "gene_name": "DOMON domain-containing protein FRRS1L",
  "term_id": "GO:0099072",
  "gene_symbol": "FRRS1L",
  "gene": "UniProtKB:Q9P0K9"
}